{
  "gene": "UniProtKB:Q6ZTR7",
  "term_id": "GO:0060271",
  "gene_symbol": "CIBAR2",
  "term_label": "cilium assembly",
  "gene_name": "CBY1-interacting BAR domain-containing protein 2"
}